biuret amidohydrolase activity [GO:0018750] (MF) Relationships: is a type of hydrolase activity, acting on carbon-nitrogen (but not peptide) bonds, in linear amides [GO:0016811] Sources: EC:3.5.1.84 Definition: Catalysis of the reaction: biuret + H2O = urea + CO2 + NH3.